NLRP6 inflammasome complex [GO:0140738] (cellular component) Relationships: is a type of GO:0061702 Definition: An inflammasome complex that consists of NLRP6, PYCARD/ASC and caspase-1 or caspase-4/caspase-11. References: PMID:30674671, PMID:34678144